{
  "gene_name": "Squamous cell carcinoma antigen recognized by T-cells 3",
  "gene_symbol": "SART3",
  "term_label": "nucleoplasm",
  "gene": "UniProtKB:Q15020",
  "term_id": "GO:0005654"
}